{
  "gene": "UniProtKB:Q99816",
  "gene_name": "Tumor susceptibility gene 101 protein",
  "term_id": "GO:0000813",
  "term_label": "ESCRT I complex",
  "gene_symbol": "TSG101"
}